{
  "gene_symbol": "GJC1",
  "gene_name": "Gap junction gamma-1 protein",
  "gene": "UniProtKB:P36383",
  "term_id": "GO:0005243",
  "term_label": "gap junction channel activity"
}